{
  "term_id": "GO:0005923",
  "gene_symbol": "CGNL1",
  "term_label": "bicellular tight junction",
  "gene_name": "Cingulin-like protein 1",
  "gene": "UniProtKB:Q0VF96"
}